{
  "gene_name": "Sterile alpha motif domain-containing protein 5",
  "gene": "UniProtKB:Q5TGI4",
  "term_id": "UNKNOWN:0003",
  "gene_symbol": "SAMD5",
  "term_label": "Unknown cellular component"
}